{
  "term_id": "UNKNOWN:0001",
  "gene_symbol": "TMEM214",
  "gene": "UniProtKB:Q6NUQ4",
  "gene_name": "Transmembrane protein 214",
  "term_label": "Unknown molecular function"
}